regulation of siderophore biosynthetic process [GO:1900704] (biological process) Definition: Any process that modulates the frequency, rate or extent of siderophore biosynthetic process. Sources: GOC:TermGenie, GOC:di Also known as: regulation of siderophore anabolism, regulation of siderophore biosynthesis, regulation of siderophore formation, regulation of siderophore synthesis, regulation of siderochrome biosynthesis, regulation of siderochrome biosynthetic process, regulation of siderophore biosynthetic process, peptide formation, regulation of siderophore biosynthetic process, peptide modification Relationships: is_a regulation of secondary metabolite biosynthetic process [GO:1900376]; regulates siderophore biosynthetic process [GO:0019290] Subtypes: negative regulation of siderophore biosynthetic process [GO:1900705], positive regulation of siderophore biosynthetic process [GO:1900706], GO:1905568